inositol hexakisphosphate 4-phosphatase activity [GO:0008707] (molecular function) Relationships: is a type of GO:0004446 Also known as: 6-phytase (name based on 1L-numbering system and not 1D-numbering), phytase activity, 4-phytase activity, 6-phytase activity, myo-inositol-hexakisphosphate 6-phosphohydrolase activity, phytate 6-phosphatase activity Sources: EC:3.1.3.26 Definition: Catalysis of the reaction: myo-inositol hexakisphosphate + H2O = 1-myo-inositol 1,2,3,4,5-pentakisphosphate + phosphate.